{
  "gene": "UniProtKB:Q0VG99",
  "gene_name": "Mesoderm posterior protein 2",
  "term_label": "nucleus",
  "gene_symbol": "MESP2",
  "term_id": "GO:0005634"
}